negative regulation of glomerular filtration [GO:0003105] (biological process) Definition: Any process that stops, prevents, or reduces the frequency, rate or extent of glomerular filtration. Glomerular filtration is the process whereby blood is filtered by the glomerulus into the renal tubule. Relationships: is a type of regulation of glomerular filtration [GO:0003093]; is a type of negative regulation of multicellular organismal process [GO:0051241]; negatively regulates glomerular filtration [GO:0003094] Sources: GOC:mtg_cardio